{
  "term_id": "GO:0005200",
  "gene": "UniProtKB:Q8TC94",
  "term_label": "structural constituent of cytoskeleton",
  "gene_name": "Actin-like protein 9",
  "gene_symbol": "ACTL9"
}